{
  "term_label": "Unknown biological process",
  "term_id": "UNKNOWN:0002",
  "gene_symbol": "MSL3B",
  "gene": "UniProtKB:P0C860",
  "gene_name": "Putative male-specific lethal-3 protein-like 2"
}